{
  "term_label": "Unknown molecular function",
  "term_id": "UNKNOWN:0001",
  "gene_name": "Protein MOST-1",
  "gene": "UniProtKB:Q9NRJ1",
  "gene_symbol": "C8orf17"
}